specification of mesonephric nephron tubule identity [GO:0061282] (biological process) Definition: The process in which the tubules arranged along the proximal/distal axis of the mesonephric nephron acquire their identity. Sources: GOC:mtg_kidney_jan10 Relationships: is a type of pattern specification involved in mesonephros development [GO:0061227]; is a type of specification of nephron tubule identity [GO:0072081]; is part of proximal/distal pattern formation involved in mesonephric nephron development [GO:0061226]; is part of mesonephric nephron tubule formation [GO:0061277] Subtypes: specification of mesonephric connecting tubule identity [GO:0061281], GO:0061283, specification of mesonephric proximal tubule identity [GO:0061284]